plant-type cell wall cellulose biosynthetic process [GO:0052324] (biological process) Also known as: cell wall cellulose biosynthesis, cellulose biosynthesis during cell wall biosynthesis Definition: The chemical reactions and pathways resulting in the formation of cellulose, a linear beta1-4 glucan of molecular mass 50-400 kDa with the pyranose units in the -4C1 conformation, as part of the organization and biogenesis of the cell wall. Relationships: is a type of GO:0030244; is_a cell wall beta-glucan biosynthetic process [GO:0034410]; is a type of plant-type cell wall cellulose metabolic process [GO:0052541]; is part of plant-type cell wall biogenesis [GO:0009832] Sources: GOC:ai Regulation: regulated by regulation of plant-type cell wall cellulose biosynthetic process [GO:2001009]; negatively regulated by negative regulation of plant-type cell wall cellulose biosynthetic process [GO:2001010]; positively regulated by positive regulation of plant-type cell wall cellulose biosynthetic process [GO:2001011]